negative regulation of epithelial cell migration [GO:0010633] (biological process) Definition: Any process that stops, prevents, or reduces the frequency, rate or extent of epithelial cell migration. Sources: GOC:BHF, GOC:dph, GOC:tb Relationships: is a type of regulation of epithelial cell migration [GO:0010632]; is a type of negative regulation of cell migration [GO:0030336]; is a type of negative regulation of multicellular organismal process [GO:0051241]; negatively regulates GO:0010631 Subtypes: negative regulation of keratinocyte migration [GO:0051548], negative regulation of border follicle cell migration [GO:1903687]